regulation of vascular wound healing [GO:0061043] (biological process) Subtypes: positive regulation of vascular wound healing [GO:0035470], negative regulation of vascular wound healing [GO:0061044] Definition: Any process that modulates the rate, frequency, or extent of blood vessel formation when new vessels emerge from the proliferation of pre-existing blood vessels and contribute to the series of events that restore integrity to damaged vasculature. Sources: GOC:dph Relationships: is a type of regulation of angiogenesis [GO:0045765]; is a type of regulation of wound healing [GO:0061041]; regulates vascular wound healing [GO:0061042]